{
  "gene": "UniProtKB:P09619",
  "gene_name": "Platelet-derived growth factor receptor beta",
  "gene_symbol": "PDGFRB",
  "term_id": "GO:0005886",
  "term_label": "plasma membrane"
}